{
  "gene_name": "Apoptosis-associated speck-like protein containing a CARD",
  "gene_symbol": "PYCARD",
  "term_id": "GO:0140608",
  "gene": "UniProtKB:Q9ULZ3",
  "term_label": "cysteine-type endopeptidase activator activity"
}